{
  "gene": "UniProtKB:O95835",
  "gene_symbol": "LATS1",
  "term_id": "GO:0000082",
  "gene_name": "Serine_threonine-protein kinase LATS1",
  "term_label": "G1/S transition of mitotic cell cycle"
}